{
  "gene_symbol": "MYH6",
  "term_label": "myosin II complex",
  "gene": "UniProtKB:P13533",
  "term_id": "GO:0016460",
  "gene_name": "Myosin-6"
}